{
  "term_id": "GO:0032332",
  "gene_name": "Transcription factor SOX-6",
  "term_label": "positive regulation of chondrocyte differentiation",
  "gene_symbol": "SOX6",
  "gene": "UniProtKB:P35712"
}